{
  "term_id": "UNKNOWN:0003",
  "term_label": "Unknown cellular component",
  "gene": "UniProtKB:Q7Z422",
  "gene_name": "SUZ domain-containing protein 1",
  "gene_symbol": "SZRD1"
}